regulation of mRNA alternative polyadenylation [GO:0140408] (biological process) References: PMID:29507755 Relationships: is a type of regulation of mRNA 3'-end processing [GO:0031440]; regulates GO:0110104 Definition: Any process that modulates the frequency, rate or extent of mRNA alternative polyadenylation. Subtypes: GO:0140409